FHL3-CREB complex [GO:0034981] (cellular component) Definition: A protein complex that contains CREB and FHL3, and is involved in transcriptional regulation. Relationships: is a type of GO:0033202; is a type of GO:0140513 References: PMID:11046156